{
  "gene_symbol": "PPTC7",
  "gene": "UniProtKB:Q8NI37",
  "gene_name": "Protein phosphatase PTC7 homolog",
  "term_id": "GO:0010795",
  "term_label": "regulation of ubiquinone biosynthetic process"
}